{
  "term_label": "cholesterol metabolic process",
  "term_id": "GO:0008203",
  "gene": "UniProtKB:P19099",
  "gene_symbol": "CYP11B2",
  "gene_name": "Cytochrome P450 11B2, mitochondrial"
}